{
  "gene_name": "BTB_POZ domain-containing protein KCTD16",
  "term_id": "UNKNOWN:0001",
  "gene": "UniProtKB:Q68DU8",
  "term_label": "Unknown molecular function",
  "gene_symbol": "KCTD16"
}